{
  "gene_symbol": "DEAF1",
  "gene": "UniProtKB:O75398",
  "term_label": "regulation of transcription by RNA polymerase II",
  "term_id": "GO:0006357",
  "gene_name": "Deformed epidermal autoregulatory factor 1 homolog"
}